{
  "gene_name": "B-cell antigen receptor complex-associated protein beta chain",
  "term_id": "GO:0009897",
  "gene": "UniProtKB:P40259",
  "term_label": "external side of plasma membrane",
  "gene_symbol": "CD79B"
}